{
  "gene_name": "Lariat debranching enzyme",
  "gene_symbol": "DBR1",
  "gene": "UniProtKB:Q9UK59",
  "term_id": "GO:0000398",
  "term_label": "mRNA splicing, via spliceosome"
}